glomerulus morphogenesis [GO:0072102] (biological process) Definition: The process in which the anatomical structures of the glomerulus are generated and organized. The glomerulus is a capillary tuft surrounded by Bowman's capsule in nephrons of the vertebrate kidney. Subtypes: GO:0035775, mesonephric glomerulus morphogenesis [GO:0061234], metanephric glomerulus morphogenesis [GO:0072275] Sources: GOC:mtg_kidney_jan10 Relationships: is a type of GO:0009653; is part of glomerulus development [GO:0032835]